{
  "term_id": "GO:0003682",
  "gene": "UniProtKB:Q76L83",
  "gene_name": "Putative Polycomb group protein ASXL2",
  "gene_symbol": "ASXL2",
  "term_label": "chromatin binding"
}